{
  "term_id": "UNKNOWN:0002",
  "gene_name": "Transmembrane protein 179B",
  "term_label": "Unknown biological process",
  "gene": "UniProtKB:Q7Z7N9",
  "gene_symbol": "TMEM179B"
}